{
  "gene_symbol": "GSN",
  "gene_name": "Gelsolin",
  "term_label": "extracellular space",
  "term_id": "GO:0005615",
  "gene": "UniProtKB:P06396"
}